negative regulation of testosterone secretion [GO:2000844] (biological process) Definition: Any process that stops, prevents or reduces the frequency, rate or extent of testosterone secretion. Sources: GOC:sl Relationships: is a type of negative regulation of lipid transport [GO:0032369]; is a type of negative regulation of hormone secretion [GO:0046888]; is_a GO:2000843; negatively regulates testosterone secretion [GO:0035936]